{
  "term_id": "GO:0010916",
  "gene": "UniProtKB:P30533",
  "gene_name": "Alpha-2-macroglobulin receptor-associated protein",
  "gene_symbol": "LRPAP1",
  "term_label": "negative regulation of very-low-density lipoprotein particle clearance"
}